dendritic shaft [GO:0043198] (cellular component) Sources: GOC:nln Relationships: is a type of cellular anatomical structure [GO:0110165]; is part of dendrite [GO:0030425] Definition: Cylindric portion of the dendrite, directly stemming from the perikaryon, and carrying the dendritic spines. Also known as: trunk